{
  "gene_name": "Olfactory receptor 4M2",
  "gene_symbol": "OR4M2",
  "gene": "UniProtKB:Q8NGB6",
  "term_id": "GO:0004984",
  "term_label": "olfactory receptor activity"
}